{
  "gene": "UniProtKB:Q96PB7",
  "gene_symbol": "OLFM3",
  "gene_name": "Noelin-3",
  "term_label": "extracellular space",
  "term_id": "GO:0005615"
}